regulation of metaphase/anaphase transition of meiosis I [GO:1905186] (biological process) Also known as: regulation of meiosis I metaphase/anaphase transition, regulation of first meiotic metaphase/anaphase transition Subtypes: GO:1905187, positive regulation of metaphase/anaphase transition of meiosis I [GO:1905188] Relationships: is a type of regulation of metaphase/anaphase transition of meiotic cell cycle [GO:1902102]; regulates GO:1990949 References: PMID:21389117 Sources: GOC:TermGenie, GO_REF:0000058 Definition: Any process that modulates the frequency, rate or extent of metaphase/anaphase transition of meiosis I.